{
  "term_id": "GO:0071040",
  "gene": "UniProtKB:Q01780",
  "gene_symbol": "EXOSC10",
  "term_label": "nuclear polyadenylation-dependent antisense transcript catabolic process",
  "gene_name": "Exosome component 10"
}